{
  "gene_name": "Epoxide hydrolase 3",
  "gene": "UniProtKB:Q9H6B9",
  "term_id": "GO:0016787",
  "term_label": "hydrolase activity",
  "gene_symbol": "EPHX3"
}